melibiose transmembrane transporter activity [GO:0015156] (molecular function) Relationships: is a type of disaccharide transmembrane transporter activity [GO:0015154]; is part of melibiose transport [GO:0015769] Definition: Enables the transfer of melibiose from one side of a membrane to the other. Melibiose is the disaccharide 6-O-alpha-D-galactopyranosyl-D-glucose and occurs as a constituent of the trisaccharide raffinose or in the exudates and nectaries of a number of plants. Subtypes: melibiose:monoatomic cation symporter activity [GO:0015487] Sources: GOC:mtg_transport, ISBN:0198506732, ISBN:0815340729